{
  "gene_symbol": "AMIGO1",
  "term_label": "brain development",
  "term_id": "GO:0007420",
  "gene_name": "Amphoterin-induced protein 1",
  "gene": "UniProtKB:Q86WK6"
}